{
  "term_id": "GO:0005783",
  "gene": "UniProtKB:Q49AH0",
  "gene_name": "Cerebral dopamine neurotrophic factor",
  "term_label": "endoplasmic reticulum",
  "gene_symbol": "CDNF"
}